{
  "term_label": "estrogen response element binding",
  "gene_symbol": "NR6A1",
  "gene_name": "Nuclear receptor subfamily 6 group A member 1",
  "term_id": "GO:0034056",
  "gene": "UniProtKB:Q15406"
}